{
  "term_id": "UNKNOWN:0002",
  "gene": "UniProtKB:Q9Y5J9",
  "gene_symbol": "TIMM8B",
  "gene_name": "Mitochondrial import inner membrane translocase subunit Tim8 B",
  "term_label": "Unknown biological process"
}